nuclear-transcribed mRNA catabolic process, nonsense-mediated decay [GO:0000184] (biological process) Definition: The nonsense-mediated decay pathway for nuclear-transcribed mRNAs degrades mRNAs in which an amino-acid codon has changed to a nonsense codon; this prevents the translation of such mRNAs into truncated, and potentially harmful, proteins. Also known as: mRNA breakdown, nonsense-mediated decay, mRNA catabolic process, nonsense-mediated, mRNA catabolism, nonsense-mediated, mRNA degradation, nonsense-mediated decay, nonsense-mediated mRNA decay, nuclear mRNA catabolic process, nonsense-mediated decay Regulation: regulated by regulation of nuclear-transcribed mRNA catabolic process, nonsense-mediated decay [GO:2000622]; negatively regulated by negative regulation of nuclear-transcribed mRNA catabolic process, nonsense-mediated decay [GO:2000623]; positively regulated by positive regulation of nuclear-transcribed mRNA catabolic process, nonsense-mediated decay [GO:2000624] Subtypes: nuclear-transcribed mRNA catabolic process, 3'-5' exonucleolytic nonsense-mediated decay [GO:0070478], GO:0070479 Relationships: is a type of nuclear-transcribed mRNA catabolic process [GO:0000956] References: PMID:10025395 Sources: GOC:krc, GOC:ma